{
  "gene_name": "Myoglobin",
  "gene_symbol": "MB",
  "term_label": "oxygen transport",
  "term_id": "GO:0015671",
  "gene": "UniProtKB:P02144"
}